{
  "gene": "UniProtKB:O75594",
  "gene_name": "Peptidoglycan recognition protein 1",
  "term_id": "GO:0016019",
  "term_label": "peptidoglycan immune receptor activity",
  "gene_symbol": "PGLYRP1"
}